tear secretion [GO:0070075] (biological process) Sources: GOC:rph Definition: The regulated release of the aqueous layer of the tear film from the lacrimal glands. Tears are the liquid product of a process of lacrimation to clean and lubricate the eyes. Tear fluid contains water, mucin, lipids, lysozyme, lactoferrin, lipocalin, lacritin, immunoglobulins, glucose, urea, sodium, and potassium. Relationships: is a type of body fluid secretion [GO:0007589]; is_a secretion by tissue [GO:0032941]